pelvic fin development [GO:0033340] (biological process) Definition: The process whose specific outcome is the progression of the pelvic fin over time, from its formation to the mature structure. Relationships: is a type of fin development [GO:0033333]; is_a GO:0060173 Sources: GOC:dgh